{
  "gene_name": "Carbonic anhydrase 13",
  "gene": "UniProtKB:Q8N1Q1",
  "term_label": "carbonate dehydratase activity",
  "gene_symbol": "CA13",
  "term_id": "GO:0004089"
}